{
  "gene": "UniProtKB:O15511",
  "gene_symbol": "ARPC5",
  "gene_name": "Actin-related protein 2_3 complex subunit 5",
  "term_id": "GO:0030674",
  "term_label": "protein-macromolecule adaptor activity"
}